jasmonic acid metabolic process [GO:0009694] (biological process) Subtypes: jasmonic acid biosynthetic process [GO:0009695] Also known as: jasmonic acid metabolism Sources: ISBN:0387969845 Relationships: is a type of GO:0001676 Definition: The chemical reactions and pathways involving jasmonic acid, a fatty acid derivative with the formula (1R-(1 alpha, 2 beta(Z)))-3-oxo-2-(2-pentenyl)cyclopentaneacetic acid. Regulation: regulated by GO:0080140